{
  "gene": "UniProtKB:O60391",
  "gene_name": "Glutamate receptor ionotropic, NMDA 3B",
  "term_label": "plasma membrane",
  "term_id": "GO:0005886",
  "gene_symbol": "GRIN3B"
}